{
  "gene": "UniProtKB:P53597",
  "term_label": "succinate-CoA ligase (ADP-forming) activity",
  "gene_symbol": "SUCLG1",
  "term_id": "GO:0004775",
  "gene_name": "Succinate--CoA ligase [ADP_GDP-forming] subunit alpha, mitochondrial"
}